{
  "term_label": "transmembrane signaling receptor activity",
  "term_id": "GO:0004888",
  "gene": "UniProtKB:P43632",
  "gene_symbol": "KIR2DS4",
  "gene_name": "Killer cell immunoglobulin-like receptor 2DS4"
}